positive regulation of white fat cell proliferation [GO:0070352] (biological process) Also known as: positive regulation of white adipocyte proliferation, positive regulation of white adipose cell proliferation, up regulation of white fat cell proliferation, up-regulation of white fat cell proliferation, upregulation of white fat cell proliferation, activation of white fat cell proliferation, stimulation of white fat cell proliferation Definition: Any process that activates or increases the rate or extent of white fat cell proliferation. Sources: GOC:mah, GOC:sl Relationships: is a type of positive regulation of fat cell proliferation [GO:0070346]; is a type of regulation of white fat cell proliferation [GO:0070350]; positively regulates GO:0070343